{
  "term_id": "GO:0003690",
  "gene_name": "Histone H1.4",
  "gene": "UniProtKB:P10412",
  "gene_symbol": "H1-4",
  "term_label": "double-stranded DNA binding"
}